leukocyte adhesion to vascular endothelial cell [GO:0061756] (biological process) Definition: The attachment of a leukocyte to vascular endothelial cell via adhesion molecules. Regulation: regulated by GO:1904994; negatively regulated by negative regulation of leukocyte adhesion to vascular endothelial cell [GO:1904995]; positively regulated by positive regulation of leukocyte adhesion to vascular endothelial cell [GO:1904996] Subtypes: GO:0036339, leukocyte tethering or rolling [GO:0050901], leukocyte activation-dependent arrest [GO:0050903], GO:0061757 References: PMID:23897866 Sources: GOC:BHF, GOC:BHF_miRNA, GOC:add, GOC:bc Relationships: is a type of leukocyte cell-cell adhesion [GO:0007159]